CTPase activity [GO:0043273] (molecular function) Definition: Catalysis of the reaction: CTP + H2O = CDP + H+ + phosphate. May or may not be coupled to another reaction. Sources: RHEA:29387 Also known as: cytidine triphosphatase activity, single-stranded DNA-dependent CTPase activity, CTPase activity, coupled Relationships: is a type of ribonucleoside triphosphate phosphatase activity [GO:0017111]